membrane protein proteolysis [GO:0033619] (biological process) Relationships: is a type of GO:0006508 Subtypes: membrane protein ectodomain proteolysis [GO:0006509], GO:0031293, membrane protein proteolysis involved in retrograde protein transport, ER to cytosol [GO:1904211] Sources: GOC:pde Definition: The proteolytic cleavage of a transmembrane protein leading to the release of its intracellular or ecto-domains.